{
  "gene_name": "Period circadian protein homolog 1",
  "gene": "UniProtKB:O15534",
  "term_id": "GO:0000122",
  "term_label": "negative regulation of transcription by RNA polymerase II",
  "gene_symbol": "PER1"
}